cellular bud [GO:0005933] (cellular component) Sources: GOC:sgd_curators Definition: A protuberance from a cell of an organism that reproduces by budding, which will grow larger and become a separate daughter cell after nuclear division, cytokinesis, and cell wall formation (when appropriate). The daughter cell may completely separate from the mother cell, or the mother and daughter cells may remain associated. Relationships: is a type of cellular anatomical structure [GO:0110165]